regulation of chondrocyte development [GO:0061181] (BP) Definition: Any process that modulates the rate, frequency, or extent of the process whose specific outcome is the progression of a chondrocyte over time, from its commitment to its mature state. Chondrocyte development does not include the steps involved in committing a chondroblast to a chondrocyte fate. Relationships: is a type of regulation of chondrocyte differentiation [GO:0032330]; is_a regulation of cell development [GO:0060284]; regulates chondrocyte development [GO:0002063] Sources: GOC:BHF, GOC:dph Subtypes: negative regulation of chondrocyte development [GO:0061182], positive regulation of chondrocyte development [GO:1902761], regulation of chondrocyte hypertrophy [GO:1903041]